{
  "term_label": "heterotrimeric G-protein complex",
  "gene_name": "Guanine nucleotide-binding protein G(olf) subunit alpha",
  "gene_symbol": "GNAL",
  "gene": "UniProtKB:P38405",
  "term_id": "GO:0005834"
}